{
  "term_id": "GO:0005789",
  "gene": "UniProtKB:Q9HCU5",
  "gene_name": "Prolactin regulatory element-binding protein",
  "gene_symbol": "PREB",
  "term_label": "endoplasmic reticulum membrane"
}